{
  "gene_name": "NEDD4 family-interacting protein 2",
  "term_label": "ubiquitin-dependent protein catabolic process",
  "term_id": "GO:0006511",
  "gene_symbol": "NDFIP2",
  "gene": "UniProtKB:Q9NV92"
}